{
  "gene": "UniProtKB:Q16254",
  "gene_symbol": "E2F4",
  "term_label": "regulation of transcription by RNA polymerase II",
  "term_id": "GO:0006357",
  "gene_name": "Transcription factor E2F4"
}